{
  "gene_name": "Synaptojanin-2",
  "term_id": "GO:0098793",
  "gene": "UniProtKB:O15056",
  "term_label": "presynapse",
  "gene_symbol": "SYNJ2"
}